{
  "gene_symbol": "OR5D16",
  "term_id": "GO:0007608",
  "term_label": "sensory perception of smell",
  "gene_name": "Olfactory receptor 5D16",
  "gene": "UniProtKB:Q8NGK9"
}